{
  "term_id": "UNKNOWN:0001",
  "gene": "UniProtKB:Q71SY5",
  "term_label": "Unknown molecular function",
  "gene_name": "Mediator of RNA polymerase II transcription subunit 25",
  "gene_symbol": "MED25"
}